{
  "gene": "UniProtKB:O95352",
  "term_label": "mitophagy",
  "term_id": "GO:0000423",
  "gene_symbol": "ATG7",
  "gene_name": "Ubiquitin-like modifier-activating enzyme ATG7"
}